{
  "term_label": "endoplasmic reticulum to Golgi vesicle-mediated transport",
  "gene_symbol": "TRAPPC3L",
  "gene_name": "Trafficking protein particle complex subunit 3-like protein",
  "gene": "UniProtKB:Q5T215",
  "term_id": "GO:0006888"
}